{
  "term_id": "GO:0007165",
  "gene": "UniProtKB:P63104",
  "gene_symbol": "YWHAZ",
  "gene_name": "14-3-3 protein zeta_delta",
  "term_label": "signal transduction"
}